{
  "gene": "UniProtKB:O60330",
  "term_id": "GO:0005886",
  "term_label": "plasma membrane",
  "gene_symbol": "PCDHGA12",
  "gene_name": "Protocadherin gamma-A12"
}